{
  "term_label": "DNA-binding transcription factor activity, RNA polymerase II-specific",
  "term_id": "GO:0000981",
  "gene": "UniProtKB:A6NFI3",
  "gene_symbol": "ZNF316",
  "gene_name": "Zinc finger protein 316"
}